{
  "gene_symbol": "NHLH2",
  "gene_name": "Helix-loop-helix protein 2",
  "gene": "UniProtKB:Q02577",
  "term_label": "DNA-binding transcription factor activity, RNA polymerase II-specific",
  "term_id": "GO:0000981"
}